{
  "gene_symbol": "RIN2",
  "gene_name": "Ras and Rab interactor 2",
  "term_label": "cytosol",
  "gene": "UniProtKB:Q8WYP3",
  "term_id": "GO:0005829"
}